{
  "term_label": "ruffle membrane",
  "gene_symbol": "PLEKHO1",
  "gene_name": "Pleckstrin homology domain-containing family O member 1",
  "gene": "UniProtKB:Q53GL0",
  "term_id": "GO:0032587"
}